{
  "gene_symbol": "HOOK3",
  "term_label": "cytoskeleton-dependent intracellular transport",
  "term_id": "GO:0030705",
  "gene": "UniProtKB:Q86VS8",
  "gene_name": "Protein Hook homolog 3"
}